translation initiation complex [GO:0070992] (cellular component) Relationships: is a type of GO:1990904; is part of cytoplasm [GO:0005737] Subtypes: eukaryotic 80S initiation complex [GO:0033291], mitochondrial translation initiation complex [GO:0180052] Definition: A ribonucleoprotein complex that contains a ribosome, mRNA, and initiator tRNA; the functional ribosome is at the AUG, with the methionyl/formyl-methionyl-tRNA positioned at the P site. Sources: GOC:hjd, GOC:mah